{
  "term_id": "GO:0005737",
  "gene_symbol": "KLHL31",
  "gene": "UniProtKB:Q9H511",
  "gene_name": "Kelch-like protein 31",
  "term_label": "cytoplasm"
}